regulation of lymphangiogenesis [GO:1901490] (biological process) Subtypes: negative regulation of lymphangiogenesis [GO:1901491], positive regulation of lymphangiogenesis [GO:1901492] References: PMID:20133819 Sources: GOC:TermGenie, GOC:dph Definition: Any process that modulates the frequency, rate or extent of lymphangiogenesis. Relationships: is a type of regulation of anatomical structure morphogenesis [GO:0022603]; regulates lymphangiogenesis [GO:0001946] Also known as: regulation of lymph vessel formation